{
  "gene_name": "Putative protein FRMPD2-like",
  "gene_symbol": "FRMPD2B",
  "term_label": "Unknown cellular component",
  "gene": "UniProtKB:Q6IN97",
  "term_id": "UNKNOWN:0003"
}